nitrobenzene catabolic process [GO:1900998] (biological process) Sources: GOC:TermGenie, GOC:yaf, UniPathway:UPA00923 Definition: The chemical reactions and pathways resulting in the breakdown of nitrobenzene. Also known as: nitrobenzene breakdown, nitrobenzene catabolism, nitrobenzene degradation Relationships: is a type of catabolic process [GO:0009056]; is a type of nitrobenzene metabolic process [GO:0018916]